{
  "gene": "UniProtKB:Q12788",
  "term_label": "endonucleolytic cleavage in 5'-ETS of tricistronic rRNA transcript (SSU-rRNA, 5.8S rRNA, LSU-rRNA)",
  "term_id": "GO:0000480",
  "gene_name": "Transducin beta-like protein 3",
  "gene_symbol": "TBL3"
}